{
  "term_label": "growth factor activity",
  "gene": "UniProtKB:O60542",
  "gene_symbol": "PSPN",
  "gene_name": "Persephin",
  "term_id": "GO:0008083"
}